o-xylene catabolic process [GO:0042186] (biological process) Sources: GOC:jl Relationships: is a type of xylene catabolic process [GO:0042184] Definition: The chemical reactions and pathways resulting in the breakdown of o-xylene, (1,2-dimethylbenzene) a colorless, liquid aromatic hydrocarbon. Also known as: o-xylene breakdown, o-xylene catabolism, o-xylene degradation, ortho-xylene catabolic process, ortho-xylene catabolism